4-nitrotoluene catabolic process [GO:0019258] (biological process) Also known as: 4-nitrotoluene breakdown, 4-nitrotoluene catabolism, 4-nitrotoluene degradation, 4NT catabolic process, 4NT catabolism Definition: The chemical reactions and pathways resulting in the breakdown of 4-nitrotoluene, 1-methyl-4-nitrobenzene. Relationships: is a type of nitrotoluene catabolic process [GO:0046263] Sources: GOC:ai